{
  "gene": "UniProtKB:Q15345",
  "gene_name": "Leucine-rich repeat-containing protein 41",
  "gene_symbol": "LRRC41",
  "term_label": "Unknown biological process",
  "term_id": "UNKNOWN:0002"
}